regulation of renal sodium excretion [GO:0035813] (biological process) Sources: GOC:mtg_25march11, GOC:yaf Subtypes: negative regulation of renal sodium excretion [GO:0035814], GO:0035815 Definition: Any process that modulates the amount of sodium excreted in urine over a unit of time. Relationships: is a type of regulation of excretion [GO:0044062]; is a type of regulation of renal system process [GO:0098801]; regulates renal sodium excretion [GO:0035812]